 [go#chebi:ph7:3] Note: Rhea list of ChEBI terms representing the major species at pH 7.3.